plant-type cell wall organization or biogenesis [GO:0071669] (biological process) Definition: A process that results in the biosynthesis of constituent macromolecules, assembly, arrangement of constituent parts, or disassembly of a cellulose- and pectin-containing cell wall. Relationships: is a type of GO:0071554 Subtypes: plant-type cell wall organization [GO:0009664], plant-type cell wall biogenesis [GO:0009832] Sources: GOC:ecd, GOC:mah Also known as: plant-type cell wall organisation or biogenesis, plant-type cell wall organization and biogenesis Regulation: regulated by GO:0080157